{
  "gene": "UniProtKB:A6NKL6",
  "gene_name": "Transmembrane protein 200C",
  "term_label": "Unknown biological process",
  "term_id": "UNKNOWN:0002",
  "gene_symbol": "TMEM200C"
}